{
  "gene_symbol": "ITGB6",
  "term_label": "cell migration",
  "term_id": "GO:0016477",
  "gene_name": "Integrin beta-6",
  "gene": "UniProtKB:P18564"
}